{
  "gene": "UniProtKB:Q9GZK6",
  "gene_symbol": "OR2J1",
  "gene_name": "Olfactory receptor 2J1",
  "term_id": "GO:0004984",
  "term_label": "olfactory receptor activity"
}